{
  "gene_symbol": "KIF2A",
  "gene": "UniProtKB:O00139",
  "term_id": "GO:0005813",
  "term_label": "centrosome",
  "gene_name": "Kinesin-like protein KIF2A"
}